{
  "gene_symbol": "SF3B1",
  "term_label": "U2 snRNP",
  "gene_name": "Splicing factor 3B subunit 1",
  "gene": "UniProtKB:O75533",
  "term_id": "GO:0005686"
}